{
  "gene": "UniProtKB:Q9Y233",
  "term_id": "GO:0004118",
  "gene_symbol": "PDE10A",
  "gene_name": "cAMP and cAMP-inhibited cGMP 3',5'-cyclic phosphodiesterase 10A",
  "term_label": "3',5'-cGMP-stimulated cyclic-nucleotide phosphodiesterase activity"
}